{
  "gene_symbol": "ZNF114",
  "gene": "UniProtKB:Q8NC26",
  "term_id": "UNKNOWN:0003",
  "term_label": "Unknown cellular component",
  "gene_name": "Zinc finger protein 114"
}